epithelial cell migration involved in mesonephric proximal tubule morphogenesis [GO:0061280] (biological process) Sources: GOC:mtg_kidney_jan10 Relationships: is a type of GO:0061278; is a type of epithelial cell migration involved in proximal tubule morphogenesis [GO:0072159]; is part of mesonephric proximal tubule morphogenesis [GO:0061276] Definition: The orderly movement of epithelial cells within a renal tubule that contributes to mesonephric proximal tubule morphogenesis.